{
  "gene_name": "Large ribosomal subunit protein bL21m",
  "term_label": "mitochondrial large ribosomal subunit",
  "term_id": "GO:0005762",
  "gene": "UniProtKB:Q7Z2W9",
  "gene_symbol": "MRPL21"
}